{
  "term_id": "GO:0006111",
  "term_label": "regulation of gluconeogenesis",
  "gene_symbol": "TCF7L2",
  "gene_name": "Transcription factor 7-like 2",
  "gene": "UniProtKB:Q9NQB0"
}